{
  "term_id": "GO:0016323",
  "gene_name": "Aquaporin-3",
  "gene": "UniProtKB:Q92482",
  "gene_symbol": "AQP3",
  "term_label": "basolateral plasma membrane"
}